{
  "gene_name": "2'-5'-oligoadenylate synthase 3",
  "term_label": "negative regulation of viral genome replication",
  "gene": "UniProtKB:Q9Y6K5",
  "gene_symbol": "OAS3",
  "term_id": "GO:0045071"
}